{
  "gene": "UniProtKB:P09525",
  "term_id": "GO:0012506",
  "gene_name": "Annexin A4",
  "gene_symbol": "ANXA4",
  "term_label": "vesicle membrane"
}